positive regulation of serotonin biosynthetic process [GO:1905629] (biological process) Definition: Any process that activates or increases the frequency, rate or extent of serotonin biosynthetic process. References: PMID:25642596 Sources: GOC:PARL, GOC:TermGenie, GOC:pad, GO_REF:0000058 Also known as: positive regulation of serotonin anabolism, positive regulation of serotonin biosynthesis, positive regulation of serotonin formation, positive regulation of serotonin synthesis, up regulation of serotonin anabolism, up regulation of serotonin biosynthesis, up regulation of serotonin biosynthetic process, up regulation of serotonin formation, up regulation of serotonin synthesis, up-regulation of serotonin anabolism, up-regulation of serotonin biosynthesis, up-regulation of serotonin biosynthetic process, up-regulation of serotonin formation, up-regulation of serotonin synthesis, upregulation of serotonin anabolism, upregulation of serotonin biosynthesis, upregulation of serotonin biosynthetic process, upregulation of serotonin formation, upregulation of serotonin synthesis, activation of serotonin anabolism, activation of serotonin biosynthesis, activation of serotonin biosynthetic process, activation of serotonin formation, activation of serotonin synthesis Relationships: is a type of positive regulation of biosynthetic process [GO:0009891]; is a type of regulation of serotonin biosynthetic process [GO:1905627]; positively regulates serotonin biosynthetic process [GO:0042427]